{
  "term_id": "GO:0005615",
  "gene_symbol": "SEMA3C",
  "gene": "UniProtKB:Q99985",
  "term_label": "extracellular space",
  "gene_name": "Semaphorin-3C"
}